{
  "gene_name": "Glycerol-3-phosphate acyltransferase 2, mitochondrial",
  "term_label": "triglyceride biosynthetic process",
  "gene": "UniProtKB:Q6NUI2",
  "gene_symbol": "GPAT2",
  "term_id": "GO:0019432"
}